negative regulation of hydrogen sulfide biosynthetic process [GO:1904827] (biological process) Also known as: down regulation of hydrogen sulfide anabolism, down regulation of hydrogen sulfide biosynthesis, down regulation of hydrogen sulfide biosynthetic process, down regulation of hydrogen sulfide formation, down regulation of hydrogen sulfide synthesis, down regulation of hydrogen sulphide biosynthesis, down regulation of hydrogen sulphide biosynthetic process, down-regulation of hydrogen sulfide anabolism, down-regulation of hydrogen sulfide biosynthesis, down-regulation of hydrogen sulfide biosynthetic process, down-regulation of hydrogen sulfide formation, down-regulation of hydrogen sulfide synthesis, down-regulation of hydrogen sulphide biosynthesis, down-regulation of hydrogen sulphide biosynthetic process, downregulation of hydrogen sulfide anabolism, downregulation of hydrogen sulfide biosynthesis, downregulation of hydrogen sulfide biosynthetic process, downregulation of hydrogen sulfide formation, downregulation of hydrogen sulfide synthesis, downregulation of hydrogen sulphide biosynthesis, downregulation of hydrogen sulphide biosynthetic process, negative regulation of hydrogen sulfide anabolism, negative regulation of hydrogen sulfide biosynthesis, negative regulation of hydrogen sulfide formation, negative regulation of hydrogen sulfide synthesis, negative regulation of hydrogen sulphide biosynthesis, negative regulation of hydrogen sulphide biosynthetic process, inhibition of hydrogen sulfide anabolism, inhibition of hydrogen sulfide biosynthesis, inhibition of hydrogen sulfide biosynthetic process, inhibition of hydrogen sulfide formation, inhibition of hydrogen sulfide synthesis, inhibition of hydrogen sulphide biosynthesis, inhibition of hydrogen sulphide biosynthetic process Definition: Any process that stops, prevents or reduces the frequency, rate or extent of hydrogen sulfide biosynthetic process. Relationships: is a type of negative regulation of biosynthetic process [GO:0009890]; is a type of GO:1904826; negatively regulates hydrogen sulfide biosynthetic process [GO:0070814] References: PMID:22034194 Sources: GOC:BHF, GOC:BHF_miRNA, GOC:TermGenie, GOC:rph, GO_REF:0000058